{
  "gene": "UniProtKB:Q8IUK8",
  "gene_symbol": "CBLN2",
  "gene_name": "Cerebellin-2",
  "term_id": "GO:0005615",
  "term_label": "extracellular space"
}